{
  "term_label": "positive regulation of oligodendrocyte differentiation",
  "gene_name": "Tumor necrosis factor receptor superfamily member 1B",
  "gene": "UniProtKB:P20333",
  "term_id": "GO:0048714",
  "gene_symbol": "TNFRSF1B"
}